{
  "gene_symbol": "PRNP",
  "gene": "UniProtKB:P04156",
  "term_label": "positive regulation of calcium-mediated signaling",
  "gene_name": "Major prion protein",
  "term_id": "GO:0050850"
}